{
  "term_id": "UNKNOWN:0001",
  "gene": "UniProtKB:Q8NBB2",
  "gene_symbol": "ST20-AS1",
  "term_label": "Unknown molecular function",
  "gene_name": "Putative uncharacterized protein ST20-AS1"
}